Cdc42 protein signal transduction [GO:0032488] (biological process) Regulation: regulated by regulation of Cdc42 protein signal transduction [GO:0032489] Definition: An intracellular signaling cassette in which a small monomeric GTPase of the Cdc42 subfamily relays a signal. References: PMID:18558478 Sources: GOC:mah Relationships: is_a Rho protein signal transduction [GO:0007266] Also known as: Cdc42 signaling, Cdc42 signaling pathway, cdc42 signalling pathway